{
  "term_id": "GO:0070885",
  "gene": "UniProtKB:Q99653",
  "gene_symbol": "CHP1",
  "term_label": "negative regulation of calcineurin-NFAT signaling cascade",
  "gene_name": "Calcineurin B homologous protein 1"
}